{
  "gene_symbol": "NUP214",
  "gene_name": "Nuclear pore complex protein Nup214",
  "term_label": "nuclear localization sequence binding",
  "gene": "UniProtKB:P35658",
  "term_id": "GO:0008139"
}